secretory vesicle [GO:0099503] (cellular component) Definition: A cytoplasmic, membrane bound vesicle that is capable of fusing to the plasma membrane to release its contents into the extracellular space. Sources: GOC:dos Relationships: is a type of GO:0031410 Subtypes: secretory granule [GO:0030141], GO:0070382